{
  "term_id": "GO:0007165",
  "gene_name": "Ras association domain-containing protein 4",
  "gene": "UniProtKB:Q9H2L5",
  "term_label": "signal transduction",
  "gene_symbol": "RASSF4"
}